{
  "gene_name": "DnaJ homolog subfamily C member 5B",
  "gene_symbol": "DNAJC5B",
  "term_id": "UNKNOWN:0001",
  "gene": "UniProtKB:Q9UF47",
  "term_label": "Unknown molecular function"
}